{
  "gene_symbol": "ALG3",
  "term_label": "Unknown biological process",
  "gene_name": "Dol-P-Man:Man(5)GlcNAc(2)-PP-Dol alpha-1,3-mannosyltransferase",
  "term_id": "UNKNOWN:0002",
  "gene": "UniProtKB:Q92685"
}